{
  "gene": "UniProtKB:Q9NUQ8",
  "gene_name": "ATP-binding cassette sub-family F member 3",
  "gene_symbol": "ABCF3",
  "term_label": "Unknown cellular component",
  "term_id": "UNKNOWN:0003"
}